basal dendrite morphogenesis [GO:0150019] (biological process) Subtypes: basal dendrite arborization [GO:0150020] Relationships: is a type of dendrite morphogenesis [GO:0048813]; is part of GO:0150018 Definition: The process in which the anatomical structures of a basal dendrite are generated and organized. References: PMID:22683681 Sources: GOC:aruk, GOC:bc